{
  "term_label": "cardiac ventricle development",
  "term_id": "GO:0003231",
  "gene_name": "Transmembrane protein 65",
  "gene_symbol": "TMEM65",
  "gene": "UniProtKB:Q6PI78"
}